{
  "gene": "UniProtKB:Q7Z449",
  "term_label": "steroid metabolic process",
  "gene_symbol": "CYP2U1",
  "term_id": "GO:0008202",
  "gene_name": "Cytochrome P450 2U1"
}